{
  "term_id": "GO:0016038",
  "gene_name": "Medium-wave-sensitive opsin 3",
  "gene": "UniProtKB:P0DN78",
  "term_label": "absorption of visible light",
  "gene_symbol": "OPN1MW3"
}